{
  "gene_symbol": "ANXA2",
  "gene": "UniProtKB:P07355",
  "gene_name": "Annexin A2",
  "term_id": "GO:0005634",
  "term_label": "nucleus"
}